regulation of retrograde axon cargo transport [GO:2001017] (biological process) Subtypes: regulation of retrograde dense core granule transport [GO:1901954], negative regulation of retrograde axon cargo transport [GO:2001018], positive regulation of retrograde axon cargo transport [GO:2001019] Also known as: regulation of retrograde axonal transport Sources: GOC:obol Relationships: is a type of regulation of intracellular transport [GO:0032386]; is a type of regulation of microtubule-based movement [GO:0060632]; regulates retrograde axonal transport [GO:0008090] Definition: Any process that modulates the frequency, rate or extent of retrograde axon cargo transport.